secoisolariciresinol dehydrogenase activity [GO:0120529] (molecular function) Sources: RHEA:33887 Definition: Catalysis of the reaction: (-)-secoisolariciresinol + 2 NAD+ = (-)-matairesinol + 2 H(+) + 2 NADH. Relationships: is a type of oxidoreductase activity, acting on the CH-OH group of donors, NAD or NADP as acceptor [GO:0016616]